3-hydroxybutyryl-CoA epimerase activity [GO:0008692] (molecular function) Definition: Catalysis of the reaction: (S)-3-hydroxybutanoyl-CoA = (R)-3-hydroxybutanoyl-CoA. Also known as: 3-hydroxyacyl-CoA epimerase activity, 3-hydroxybutanoyl-CoA 3-epimerase activity, 3-hydroxybutyryl coenzyme A epimerase activity Relationships: is a type of racemase and epimerase activity, acting on hydroxy acids and derivatives [GO:0016856] Sources: EC:5.1.2.3